response to stilbenoid [GO:0035634] (biological process) Relationships: is a type of response to chemical [GO:0042221] Definition: Any process that results in a change in state or activity of a cell or an organism (in terms of movement, secretion, enzyme production, gene expression, etc.) as a result of exposure to a stilbenoid. Stilbenoids are secondary products of heartwood formation in trees that can act as phytoalexins. Stilbenoids are hydroxylated derivatives of stilbene. They belong to the family of phenylpropanoids and share most of their biosynthesis pathway with chalcones. Sources: GOC:yaf, Wikipedia:Stilbenoid Subtypes: response to resveratrol [GO:1904638]